{
  "gene": "UniProtKB:P50897",
  "gene_name": "Palmitoyl-protein thioesterase 1",
  "gene_symbol": "PPT1",
  "term_id": "GO:0008474",
  "term_label": "palmitoyl-(protein) hydrolase activity"
}